caveola assembly [GO:0070836] (biological process) Definition: The aggregation, arrangement and bonding together of a set of components to form a caveola. A caveola is a plasma membrane raft that forms a small pit, depression, or invagination that communicates with the outside of a cell and extends inward, indenting the cytoplasm and the cell membrane. Relationships: is a type of plasma membrane raft assembly [GO:0044854] Also known as: caveola formation, caveolar biogenesis References: PMID:12633858 Sources: GOC:BHF, GOC:mah, GOC:vk